{
  "term_id": "GO:0048738",
  "gene_symbol": "MYL7",
  "term_label": "cardiac muscle tissue development",
  "gene_name": "Myosin regulatory light chain 2, atrial isoform",
  "gene": "UniProtKB:Q01449"
}